mitotic spindle pole [GO:0097431] (CC) Definition: Either of the ends of a mitotic spindle, a spindle that forms as part of mitosis, where spindle microtubules are organized; usually contains a microtubule organizing center and accessory molecules, spindle microtubules and astral microtubules. Sources: GOC:vw Relationships: is a type of spindle pole [GO:0000922]; is part of GO:0072686